{
  "term_label": "heparin binding",
  "gene_name": "Protein NDNF",
  "term_id": "GO:0008201",
  "gene": "UniProtKB:Q8TB73",
  "gene_symbol": "NDNF"
}